{
  "gene_name": "Homeobox protein SIX4",
  "term_label": "regulation of transcription by RNA polymerase II",
  "term_id": "GO:0006357",
  "gene_symbol": "SIX4",
  "gene": "UniProtKB:Q9UIU6"
}